{
  "gene_name": "Sorting nexin-9",
  "gene_symbol": "SNX9",
  "term_label": "plasma membrane",
  "gene": "UniProtKB:Q9Y5X1",
  "term_id": "GO:0005886"
}